{
  "gene_name": "Centromere protein X",
  "term_label": "Unknown molecular function",
  "gene_symbol": "CENPX",
  "gene": "UniProtKB:A8MT69",
  "term_id": "UNKNOWN:0001"
}